{
  "term_id": "GO:0008017",
  "gene_symbol": "KIF5B",
  "gene_name": "Kinesin-1 heavy chain",
  "term_label": "microtubule binding",
  "gene": "UniProtKB:P33176"
}